{
  "term_id": "UNKNOWN:0002",
  "gene_symbol": "PSPHP1",
  "gene": "UniProtKB:O15172",
  "term_label": "Unknown biological process",
  "gene_name": "Putative phosphoserine phosphatase-like protein"
}